{
  "term_id": "UNKNOWN:0001",
  "term_label": "Unknown molecular function",
  "gene": "UniProtKB:Q0VG73",
  "gene_name": "Putative uncharacterized protein LOC152225",
  "gene_symbol": "Q0VG73"
}